fMet-Leu-Phe receptor binding [GO:0031761] (molecular function) Relationships: is a type of GO:0001664 Definition: Binding to a fMet-Leu-Phe receptor. Sources: GOC:mah, GOC:nln Also known as: N-formyl peptide receptor binding, fMet-Leu-Phe receptor ligand